heart trabecula formation [GO:0060347] (BP) Definition: The process of creating a trabecula in the heart. A trabecula is a tissue element in the form of a small beam, strut or rod. Also known as: cardiac trabecula formation, cardiac trabeculation, heart trabeculation, heart trabecula biogenesis Sources: GOC:dph Relationships: is a type of trabecula formation [GO:0060343]; is part of GO:0003206; is part of heart trabecula morphogenesis [GO:0061384]